{
  "gene_name": "Dual specificity protein phosphatase CDC14A",
  "term_id": "GO:0005730",
  "gene_symbol": "CDC14A",
  "gene": "UniProtKB:Q9UNH5",
  "term_label": "nucleolus"
}